{
  "gene": "UniProtKB:Q9NPG8",
  "gene_symbol": "ZDHHC4",
  "term_label": "endoplasmic reticulum",
  "term_id": "GO:0005783",
  "gene_name": "Palmitoyltransferase ZDHHC4"
}